{
  "gene_name": "Myosin-15",
  "gene": "UniProtKB:Q9Y2K3",
  "gene_symbol": "MYH15",
  "term_label": "myosin filament",
  "term_id": "GO:0032982"
}